{
  "gene": "UniProtKB:Q9NZY2",
  "gene_symbol": "FAM30A",
  "term_label": "Unknown molecular function",
  "term_id": "UNKNOWN:0001",
  "gene_name": "Putative uncharacterized protein FAM30A"
}